{
  "gene_symbol": "CFHR2",
  "gene": "UniProtKB:P36980",
  "term_label": "complement activation",
  "term_id": "GO:0006956",
  "gene_name": "Complement factor H-related protein 2"
}